{
  "gene_name": "Large ribosomal subunit protein eL14",
  "term_id": "GO:0003735",
  "term_label": "structural constituent of ribosome",
  "gene_symbol": "RPL14",
  "gene": "UniProtKB:P50914"
}